{
  "gene_symbol": "DGAT1",
  "gene": "UniProtKB:O75907",
  "gene_name": "Diacylglycerol O-acyltransferase 1",
  "term_label": "endoplasmic reticulum membrane",
  "term_id": "GO:0005789"
}